{
  "gene": "UniProtKB:Q04725",
  "term_id": "GO:0005634",
  "gene_name": "Transducin-like enhancer protein 2",
  "gene_symbol": "TLE2",
  "term_label": "nucleus"
}